protein deubiquitination involved in ubiquitin-dependent protein catabolic process [GO:0071947] (biological process) Relationships: is a type of GO:0016579; is part of GO:0006511 Sources: GOC:mah Definition: The removal of one or more ubiquitin groups from a protein as part of a process of ubiquitin-dependent protein catabolism.